{
  "gene_name": "Putative solute carrier family 22 member 31",
  "gene_symbol": "SLC22A31",
  "gene": "UniProtKB:A6NKX4",
  "term_id": "UNKNOWN:0003",
  "term_label": "Unknown cellular component"
}